{
  "term_label": "bicellular tight junction assembly",
  "gene": "UniProtKB:O95832",
  "gene_symbol": "CLDN1",
  "gene_name": "Claudin-1",
  "term_id": "GO:0070830"
}